{
  "gene_symbol": "VMP1",
  "gene": "UniProtKB:Q96GC9",
  "term_label": "autophagosome assembly",
  "term_id": "GO:0000045",
  "gene_name": "Vacuole membrane protein 1"
}